{
  "term_label": "chromosome passenger complex",
  "gene_name": "Aurora kinase A",
  "gene": "UniProtKB:O14965",
  "term_id": "GO:0032133",
  "gene_symbol": "AURKA"
}